{
  "term_label": "inositol hexakisphosphate kinase activity",
  "gene_symbol": "ITPKA",
  "gene_name": "Inositol-trisphosphate 3-kinase A",
  "gene": "UniProtKB:P23677",
  "term_id": "GO:0000828"
}